{
  "gene": "UniProtKB:P22413",
  "gene_symbol": "ENPP1",
  "gene_name": "Ectonucleotide pyrophosphatase_phosphodiesterase family member 1",
  "term_label": "nucleoside triphosphate catabolic process",
  "term_id": "GO:0009143"
}